{
  "term_label": "actin-based cell projection",
  "term_id": "GO:0098858",
  "gene_symbol": "ABI2",
  "gene": "UniProtKB:Q9NYB9",
  "gene_name": "Abl interactor 2"
}